{
  "gene_name": "Acid-sensing ion channel 2",
  "term_label": "ligand-gated sodium channel activity",
  "term_id": "GO:0015280",
  "gene_symbol": "ASIC2",
  "gene": "UniProtKB:Q16515"
}